negative regulation of calcium ion transport [GO:0051926] (biological process) Sources: GOC:ai Also known as: down regulation of calcium ion transport, down-regulation of calcium ion transport, downregulation of calcium ion transport, negative regulation of calcium transport, inhibition of calcium ion transport Subtypes: GO:0090281, GO:0106128, negative regulation of calcium ion import into sarcoplasmic reticulum [GO:1902081], negative regulation of calcium ion transmembrane transport [GO:1903170] Definition: Any process that stops, prevents, or reduces the frequency, rate or extent of the directed movement of calcium ions into, out of or within a cell, or between cells, by means of some agent such as a transporter or pore. Relationships: is a type of negative regulation of monoatomic ion transport [GO:0043271]; is a type of GO:0051924; negatively regulates GO:0006816